{
  "gene": "UniProtKB:P98173",
  "term_label": "signal transduction",
  "gene_name": "Protein FAM3A",
  "gene_symbol": "FAM3A",
  "term_id": "GO:0007165"
}